activation of membrane attack complex [GO:0001905] (biological process) Relationships: is a type of GO:0006956 Regulation: regulated by regulation of activation of membrane attack complex [GO:0001969]; positively regulated by positive regulation of activation of membrane attack complex [GO:0001970]; negatively regulated by negative regulation of activation of membrane attack complex [GO:0001971] Sources: GOC:add, ISBN:0781735149 Definition: The activation of the membrane attack complex components of the complement cascade which can result in death of a target cell through cytolysis. Also known as: MAC assembly, MAC formation, activation of MAC, membrane attack complex assembly, membrane attack complex formation, activation of TCC, activation of terminal complement complex, activation of the terminal complement cascade